sterol binding [GO:0032934] (molecular function) Subtypes: oxysterol binding [GO:0008142], cholesterol binding [GO:0015485], GO:0035100 Also known as: sterol carrier activity Definition: Binding to a sterol, a steroid containing a hydroxy group in the 3 position, closely related to cholestan-3-ol. Relationships: is a type of GO:0005496 Sources: GOC:mah